{
  "gene": "UniProtKB:P13747",
  "term_label": "extracellular space",
  "gene_name": "HLA class I histocompatibility antigen, alpha chain E",
  "term_id": "GO:0005615",
  "gene_symbol": "HLA-E"
}